positive regulation of actin filament depolymerization [GO:0030836] (biological process) Definition: Any process that activates or increases the frequency, rate or extent of actin depolymerization. Also known as: positive regulation of actin polymerization and/or depolymerization, actin filament destabilization, positive regulation of actin depolymerization, up regulation of actin filament depolymerization, up-regulation of actin filament depolymerization, upregulation of actin filament depolymerization, activation of actin filament depolymerization, stimulation of actin filament depolymerization Relationships: is a type of regulation of actin filament depolymerization [GO:0030834]; is a type of GO:0051495; is a type of positive regulation of protein depolymerization [GO:1901881]; is a type of positive regulation of supramolecular fiber organization [GO:1902905]; positively regulates actin filament depolymerization [GO:0030042] Sources: GOC:mah Note: Note that this term was split from 'positive regulation of actin polymerization and/or depolymerization ; GO:0045758' (sibling term 'positive regulation of actin polymerization ; GO:0030838'). Subtypes: GO:0051695, negative regulation of barbed-end actin filament capping [GO:2000813]